{
  "gene_name": "Homeobox protein Hox-D10",
  "gene": "UniProtKB:P28358",
  "term_id": "GO:0000978",
  "term_label": "RNA polymerase II cis-regulatory region sequence-specific DNA binding",
  "gene_symbol": "HOXD10"
}